metallopeptidase activity [GO:0008237] (molecular function) Regulation: RO_0002211 by regulation of metallopeptidase activity [GO:1905048]; negatively regulated by negative regulation of metallopeptidase activity [GO:1905049]; positively regulated by positive regulation of metallopeptidase activity [GO:1905050] Also known as: metalloprotease activity, metalloproteinase activity Definition: Catalysis of the hydrolysis of peptide bonds by a mechanism in which water acts as a nucleophile, one or two metal ions hold the water molecule in place, and charged amino acid side chains are ligands for the metal ions. Sources: GOC:mah, https://www.ebi.ac.uk/merops/about/glossary.shtml#CATTYPE Subtypes: metalloendopeptidase activity [GO:0004222], metalloexopeptidase activity [GO:0008235], metal-dependent deubiquitinase activity [GO:0140492], GO:0140758 Relationships: is a type of peptidase activity [GO:0008233]